{
  "term_id": "GO:0031643",
  "gene_name": "Cystatin-F",
  "term_label": "positive regulation of myelination",
  "gene_symbol": "CST7",
  "gene": "UniProtKB:O76096"
}